{
  "term_label": "Unknown molecular function",
  "term_id": "UNKNOWN:0001",
  "gene_name": "Immunoglobulin-like and fibronectin type III domain-containing protein 1",
  "gene": "UniProtKB:Q86VF2",
  "gene_symbol": "IGFN1"
}